{
  "gene_symbol": "ZNF615",
  "gene": "UniProtKB:Q8N8J6",
  "term_label": "nucleus",
  "gene_name": "Zinc finger protein 615",
  "term_id": "GO:0005634"
}